{
  "term_label": "Unknown cellular component",
  "gene": "UniProtKB:Q96JK4",
  "gene_name": "HHIP-like protein 1",
  "gene_symbol": "HHIPL1",
  "term_id": "UNKNOWN:0003"
}